RITS complex assembly [GO:1904802] (BP) Relationships: is a type of protein-RNA complex assembly [GO:0022618] Also known as: RITS complex formation Definition: The aggregation, arrangement and bonding together of a set of components to form a RITS complex. References: PMID:26443059 Sources: GOC:TermGenie, GO_REF:0000079